{
  "gene_symbol": "MRPL3",
  "term_label": "mitochondrial large ribosomal subunit",
  "gene_name": "Large ribosomal subunit protein uL3m",
  "gene": "UniProtKB:P09001",
  "term_id": "GO:0005762"
}